{
  "term_id": "GO:0016020",
  "term_label": "membrane",
  "gene": "UniProtKB:Q9NYW4",
  "gene_symbol": "TAS2R5",
  "gene_name": "Taste receptor type 2 member 5"
}